{
  "term_label": "nucleus",
  "gene": "UniProtKB:Q9BSD3",
  "term_id": "GO:0005634",
  "gene_name": "RAD9, HUS1, RAD1-interacting nuclear orphan protein 1",
  "gene_symbol": "RHNO1"
}